{
  "gene_name": "Microtubule-associated protein RP_EB family member 3",
  "gene": "UniProtKB:Q9UPY8",
  "term_label": "microtubule organizing center",
  "term_id": "GO:0005815",
  "gene_symbol": "MAPRE3"
}